termination of G protein-coupled receptor signaling pathway [GO:0038032] (BP) Also known as: termination of G-protein coupled receptor signaling pathway, termination of G-protein coupled receptor signalling pathway, termination of GPCR signaling pathway Relationships: is_a termination of signal transduction [GO:0023021]; is a type of negative regulation of G protein-coupled receptor signaling pathway [GO:0045744] Definition: The signaling process in which G protein-coupled receptor signaling is brought to an end. For example, through the action of GTPase-activating proteins (GAPs) that act to accelerate hydrolysis of GTP to GDP on G-alpha proteins, thereby terminating the transduced signal. Sources: GOC:bf, GOC:signaling